{
  "term_id": "GO:1990726",
  "gene_symbol": "LSM5",
  "gene_name": "U6 snRNA-associated Sm-like protein LSm5",
  "term_label": "Lsm1-7-Pat1 complex",
  "gene": "UniProtKB:Q9Y4Y9"
}